dinoflagellate antapex [GO:0097684] (cellular component) Relationships: is a type of cellular anatomical structure [GO:0110165]; BFO_0000050 GO:0097614 Subtypes: dinoflagellate antapical horn [GO:0097687] Note: The term name refers to a taxonomic group to make the label unique with respect to similarly-named anatomical structures. Sources: GOC:at, Wikipedia:Dinoflagellate#Morphology, http://tolweb.org/Dinoflagellates/2445 Definition: The anterior most point of a dinoflagellate hypocone. Also known as: antapex